protein localization to membrane [GO:0072657] (biological process) Relationships: is a type of intracellular protein localization [GO:0008104]; is_a localization within membrane [GO:0051668] Subtypes: protein localization to nuclear inner membrane [GO:0036228], receptor clustering [GO:0043113], GO:0044862, protein import into chloroplast thylakoid membrane [GO:0045038], protein import into peroxisome membrane [GO:0045046], protein localization to plasma membrane [GO:0072659], protein localization to outer membrane [GO:0089705], GO:0097117, postsynaptic density protein 95 clustering [GO:0097119], GO:0098877, GO:0099644, protein localization to prospore membrane [GO:1902657], protein localization to membrane raft [GO:1903044], protein localization to Golgi membrane [GO:1903292], protein localization to basolateral plasma membrane [GO:1903361], protein localization to plasma membrane of cell tip [GO:1903418], protein localization to ciliary membrane [GO:1903441], protein localization to postsynaptic membrane [GO:1903539], GO:1903778, protein localization to microvillus membrane [GO:1904107], GO:1905345, GO:1990656 Definition: A process in which a protein is transported to, or maintained in, a specific location in a membrane. Sources: GOC:mah Also known as: protein localisation in membrane, protein localization in membrane Regulation: regulated by regulation of protein localization to membrane [GO:1905475]; negatively regulated by negative regulation of protein localization to membrane [GO:1905476]; positively regulated by positive regulation of protein localization to membrane [GO:1905477]